acid-ammonia (or amide) ligase activity [GO:0016880] (molecular function) Also known as: amide synthase activity Sources: GOC:jl, GOC:mah Subtypes: GO:0008795, glutathionylspermidine synthase activity [GO:0008885], GO:0016211, diphthine-ammonia ligase activity [GO:0017178], glutamate-putrescine ligase activity [GO:0034024], D-aspartate ligase activity [GO:0034025], cysteine-glucosaminylinositol ligase activity [GO:0035446], adenosylcobinamide-phosphate synthase activity [GO:0043757], phosphoribosylglycinamide formyltransferase 2 activity [GO:0043815], aspartate-ammonia ligase (ADP-forming) activity [GO:0047478], trypanothione synthase activity [GO:0047479], 4-methyleneglutamate-ammonia ligase activity [GO:0047581], glutamate-ethylamine ligase activity [GO:0047942], peptidoglycan asparagine synthase activity [GO:0102115], 8-demethylnovobiocate synthase activity [GO:0102527] Relationships: is a type of ligase activity, forming carbon-nitrogen bonds [GO:0016879] Definition: Catalysis of the ligation of an acid to ammonia (NH3) or an amide via a carbon-nitrogen bond, with the concomitant hydrolysis of the diphosphate bond in ATP or a similar triphosphate.